lipoate metabolic process [GO:0009106] (biological process) Subtypes: lipoate biosynthetic process [GO:0009107], lipoate catabolic process [GO:0032323] Relationships: is a type of fatty acid metabolic process [GO:0006631]; is a type of GO:0006790 Sources: GOC:ai, ISBN:0198506732 Also known as: lipoate metabolism, lipoic acid metabolic process, lipoic acid metabolism Definition: The chemical reactions and pathways involving lipoate, 1,2-dithiolane-3-pentanoate, the anion derived from lipoic acid.